{
  "gene_name": "Aminoacylase-1",
  "gene": "UniProtKB:Q03154",
  "term_id": "UNKNOWN:0002",
  "gene_symbol": "ACY1",
  "term_label": "Unknown biological process"
}